{
  "gene_name": "Lymphocyte antigen 6D",
  "term_id": "GO:0009986",
  "gene_symbol": "LY6D",
  "gene": "UniProtKB:Q14210",
  "term_label": "cell surface"
}